{
  "gene_name": "Zinc finger protein 276",
  "term_label": "regulation of transcription by RNA polymerase II",
  "gene": "UniProtKB:Q8N554",
  "term_id": "GO:0006357",
  "gene_symbol": "ZNF276"
}